{
  "term_id": "UNKNOWN:0001",
  "gene_symbol": "NLGN2",
  "gene": "UniProtKB:Q8NFZ4",
  "term_label": "Unknown molecular function",
  "gene_name": "Neuroligin-2"
}